{
  "gene_symbol": "TECPR2",
  "term_id": "UNKNOWN:0003",
  "term_label": "Unknown cellular component",
  "gene": "UniProtKB:O15040",
  "gene_name": "Tectonin beta-propeller repeat-containing protein 2"
}